interleukin-9 receptor complex [GO:0005897] (cellular component) Definition: A protein complex that binds interleukin-9; comprises an alpha and a beta subunit. The alpha chain is specific to the interleukin-9 receptor, whereas the beta chain is shared with the receptors for several other interleukins. References: PMID:10642536 Sources: GOC:mah Also known as: IL-9 receptor complex Relationships: is a type of GO:0098802